{
  "gene_name": "Myristoylated alanine-rich C-kinase substrate",
  "gene": "UniProtKB:P29966",
  "term_id": "GO:0051015",
  "term_label": "actin filament binding",
  "gene_symbol": "MARCKS"
}